{
  "term_id": "GO:0043410",
  "term_label": "positive regulation of MAPK cascade",
  "gene": "UniProtKB:O60258",
  "gene_name": "Fibroblast growth factor 17",
  "gene_symbol": "FGF17"
}